{
  "term_label": "Unknown molecular function",
  "gene": "UniProtKB:Q96MH7",
  "term_id": "UNKNOWN:0001",
  "gene_symbol": "C5orf34",
  "gene_name": "Uncharacterized protein C5orf34"
}